{
  "gene_name": "Transmembrane protein 51",
  "term_label": "Unknown molecular function",
  "term_id": "UNKNOWN:0001",
  "gene": "UniProtKB:Q9NW97",
  "gene_symbol": "TMEM51"
}